{
  "term_id": "UNKNOWN:0002",
  "gene_name": "MORF4 family-associated protein 1",
  "term_label": "Unknown biological process",
  "gene": "UniProtKB:Q9Y605",
  "gene_symbol": "MRFAP1"
}